{
  "gene_name": "Histone H1.1",
  "term_label": "chromosome condensation",
  "gene_symbol": "H1-1",
  "term_id": "GO:0030261",
  "gene": "UniProtKB:Q02539"
}